{
  "gene": "UniProtKB:O14944",
  "term_id": "GO:0005615",
  "gene_name": "Proepiregulin",
  "gene_symbol": "EREG",
  "term_label": "extracellular space"
}